protein localization to microvillus [GO:1904106] (biological process) Also known as: protein localisation in microvillus, protein localisation to microvillus, protein localization in microvillus Subtypes: protein localization to microvillus membrane [GO:1904107] Definition: A process in which a protein is transported to, or maintained in, a location within a microvillus. Relationships: is a type of intracellular protein localization [GO:0008104] References: PMID:25335890 Sources: GOC:TermGenie, GOC:kmv, GO_REF:0000087